{
  "term_label": "Unknown molecular function",
  "term_id": "UNKNOWN:0001",
  "gene_name": "Glutathione hydrolase light chain 2",
  "gene": "UniProtKB:Q14390",
  "gene_symbol": "GGTLC2"
}